ubiquitin-like protein conjugating enzyme binding [GO:0044390] (MF) Definition: Binding to a ubiquitin-like protein conjugating enzyme such as ubiquitin conjugating enzyme. Relationships: is a type of GO:0019899 Also known as: E2 protein ligase binding, small protein conjugating enzyme binding Sources: GOC:jl Subtypes: ubiquitin conjugating enzyme binding [GO:0031624]